{
  "term_label": "nucleus",
  "gene": "UniProtKB:Q5T9G4",
  "term_id": "GO:0005634",
  "gene_name": "Armadillo repeat-containing protein 12",
  "gene_symbol": "ARMC12"
}